{
  "gene": "UniProtKB:O00291",
  "gene_name": "Huntingtin-interacting protein 1",
  "term_label": "regulation of apoptotic process",
  "gene_symbol": "HIP1",
  "term_id": "GO:0042981"
}